{
  "term_label": "Unknown cellular component",
  "term_id": "UNKNOWN:0003",
  "gene_name": "P2Y purinoceptor 12",
  "gene_symbol": "P2RY12",
  "gene": "UniProtKB:Q9H244"
}